{
  "term_id": "UNKNOWN:0002",
  "gene": "UniProtKB:Q9GZN1",
  "gene_symbol": "ACTR6",
  "term_label": "Unknown biological process",
  "gene_name": "Actin-related protein 6"
}